trehalose metabolic process [GO:0005991] (biological process) Subtypes: GO:0005992, trehalose catabolic process [GO:0005993] Also known as: mycose metabolic process, mycose metabolism, mykose metabolic process, mykose metabolism, trehalose metabolism Regulation: regulated by regulation of trehalose metabolic process [GO:0090062] Definition: The chemical reactions and pathways involving trehalose, a disaccharide that consists of two molecules of glucose and is isomeric with sucrose. Relationships: is a type of disaccharide metabolic process [GO:0005984] Sources: GOC:jl, ISBN:0028623819